{
  "term_id": "GO:0016251",
  "gene": "UniProtKB:P52657",
  "gene_symbol": "GTF2A2",
  "term_label": "RNA polymerase II general transcription initiation factor activity",
  "gene_name": "Transcription initiation factor IIA subunit 2"
}